{
  "gene": "UniProtKB:Q8NHV1",
  "gene_symbol": "GIMAP7",
  "term_id": "UNKNOWN:0003",
  "term_label": "Unknown cellular component",
  "gene_name": "GTPase IMAP family member 7"
}